{
  "gene_name": "Cell adhesion molecule DSCAM",
  "term_label": "axon",
  "term_id": "GO:0030424",
  "gene_symbol": "DSCAM",
  "gene": "UniProtKB:O60469"
}